{
  "gene_symbol": "PCDH15",
  "gene_name": "Protocadherin-15",
  "gene": "UniProtKB:Q96QU1",
  "term_label": "cell adhesion molecule binding",
  "term_id": "GO:0050839"
}